internode patterning [GO:0080006] (biological process) Definition: Determines the spacing between two shoot nodes. A shoot node is the region of the shoot where the spikelet, flower, floret, branch, bud and/or leaves are attached. Relationships: is a type of GO:0007389; is part of shoot system development [GO:0048367] Sources: GOC:tb